formation of extrachromosomal circular DNA [GO:0001325] (biological process) Subtypes: t-circle formation [GO:0090656] Relationships: is a type of DNA metabolic process [GO:0006259]; is a type of cellular component assembly [GO:0022607] Definition: Excision from the chromosome and circularization of a region of chromosomal DNA, generally, but not always, via homologous recombination between direct tandem repeats. References: PMID:12044938 Sources: GOC:jh Also known as: assembly of extrachromosomal circular DNA